{
  "term_label": "positive regulation of T cell proliferation",
  "gene_symbol": "CD274",
  "term_id": "GO:0042102",
  "gene_name": "Programmed cell death 1 ligand 1",
  "gene": "UniProtKB:Q9NZQ7"
}